{
  "term_label": "cytosol",
  "gene": "UniProtKB:Q8N335",
  "gene_symbol": "GPD1L",
  "gene_name": "Glycerol-3-phosphate dehydrogenase 1-like protein",
  "term_id": "GO:0005829"
}